{
  "gene_name": "Interleukin-2",
  "gene": "UniProtKB:P60568",
  "term_id": "GO:0002366",
  "term_label": "leukocyte activation involved in immune response",
  "gene_symbol": "IL2"
}